embryonic nail plate morphogenesis [GO:0035880] (BP) References: PMID:11369996 Sources: GOC:BHF, GOC:vk, ISBN:0323025781, UBERON:0008198, Wikipedia:Nail_(anatomy) Relationships: is a type of GO:0048598; is part of GO:0035878; is part of embryonic digit morphogenesis [GO:0042733] Definition: The process, occurring in the embryo, by which the anatomical structures of a nail plate are generated and organized. The nail plate is the hard and translucent portion of the nail, composed of keratin, and serves to protect the tips of digits.